specification of loop of Henle identity [GO:0072086] (biological process) Sources: GOC:bf, GOC:mtg_kidney_jan10 Definition: The process in which the loop of Henle of the kidney nephron acquires its identity. Relationships: is_a specification of nephron tubule identity [GO:0072081]; is part of loop of Henle development [GO:0072070] Also known as: specification of intermediate tubule identity Subtypes: specification of metanephric loop of Henle identity [GO:0072296]